{
  "gene": "UniProtKB:Q2M3R5",
  "term_label": "calcium ion export across plasma membrane",
  "gene_name": "Solute carrier family 35 member G1",
  "gene_symbol": "SLC35G1",
  "term_id": "GO:1990034"
}